{
  "term_label": "protein tyrosine kinase activator activity",
  "term_id": "GO:0030296",
  "gene_symbol": "AFAP1L2",
  "gene": "UniProtKB:Q8N4X5",
  "gene_name": "Actin filament-associated protein 1-like 2"
}